{
  "gene_symbol": "HRH1",
  "gene_name": "Histamine H1 receptor",
  "gene": "UniProtKB:P35367",
  "term_id": "GO:0004969",
  "term_label": "histamine receptor activity"
}